{
  "gene_name": "Ammonium transporter Rh type B",
  "gene_symbol": "RHBG",
  "term_id": "GO:0008519",
  "gene": "UniProtKB:Q9H310",
  "term_label": "ammonium channel activity"
}